regulation of T-helper 17 cell extravasation [GO:2000455] (biological process) Relationships: is a type of GO:2000449; regulates GO:0035699 Definition: Any process that modulates the frequency, rate or extent of T-helper 17 cell extravasation. Subtypes: GO:2000456, positive regulation of T-helper 17 cell extravasation [GO:2000457] Sources: GOC:obol